tRNA-dihydrouridine17 synthase activity [GO:0102263] (molecular function) Definition: Catalysis of the reaction: a 5,6-dihydrouracil17 in tRNA + NAD(P) = H+ + a uracil17 in tRNA + NAD(P)H. Sources: GOC:pz Relationships: is a type of tRNA dihydrouridine synthase activity [GO:0017150]